matrix metallopeptidase secretion [GO:1990773] (biological process) References: PMID:8679543 Relationships: is a type of GO:0009306 Definition: The regulated release of matrix metallopeptidases, a family of zinc-dependent endopeptidases that can degrade extracellular matrix proteins and process other types of proteins. Regulation: regulated by regulation of matrix metallopeptidase secretion [GO:1904464]; negatively regulated by GO:1904465; positively regulated by positive regulation of matrix metallopeptidase secretion [GO:1904466] Also known as: MMP secretion, matrix metalloproteinase secretion